{
  "gene": "UniProtKB:Q9BXU8",
  "gene_symbol": "FTHL17",
  "term_id": "UNKNOWN:0002",
  "term_label": "Unknown biological process",
  "gene_name": "Ferritin heavy polypeptide-like 17"
}